{
  "term_label": "chromatin binding",
  "gene": "UniProtKB:Q9ULI0",
  "gene_name": "ATPase family AAA domain-containing protein 2B",
  "term_id": "GO:0003682",
  "gene_symbol": "ATAD2B"
}